{
  "gene_name": "Transcription factor SOX-11",
  "term_label": "RNA polymerase II cis-regulatory region sequence-specific DNA binding",
  "term_id": "GO:0000978",
  "gene": "UniProtKB:P35716",
  "gene_symbol": "SOX11"
}